{
  "gene_symbol": "MAF",
  "gene_name": "Transcription factor Maf",
  "term_id": "GO:0006357",
  "gene": "UniProtKB:O75444",
  "term_label": "regulation of transcription by RNA polymerase II"
}